{
  "gene_name": "5' exonuclease Apollo",
  "gene": "UniProtKB:Q9H816",
  "term_id": "GO:0000723",
  "term_label": "telomere maintenance",
  "gene_symbol": "DCLRE1B"
}